{
  "term_id": "GO:0005634",
  "term_label": "nucleus",
  "gene": "UniProtKB:P51114",
  "gene_symbol": "FXR1",
  "gene_name": "RNA-binding protein FXR1"
}